aspartate secretion [GO:0061528] (biological process) Regulation: regulated by regulation of aspartate secretion [GO:1904448]; negatively regulated by negative regulation of aspartate secretion [GO:1904449]; positively regulated by positive regulation of aspartate secretion [GO:1904450] Subtypes: GO:0061530 Sources: GOC:dph Relationships: is_a GO:0015740; is a type of acidic amino acid transport [GO:0015800]; is a type of secretion by cell [GO:0032940]; is a type of nitrogen compound transport [GO:0071705] Definition: The regulated release of aspartate by a cell.